8-oxo-7,8-dihydroguanosine triphosphate pyrophosphatase activity [GO:0008413] (molecular function) Also known as: 7,8-dihydro-8-oxoguanine-triphosphatase activity, 8-oxo-7,8-dihydroguanine triphosphatase activity, 8-oxo-7,8-dihydroguanosine triphosphatase activity, 8-oxo-GTPase activity Definition: Catalysis of the reaction: 8-oxo-7,8-dihydroguanosine triphosphate (8-oxo-GTP) + H2O = 8-oxo-7,8-dihydroguanosine diphosphate (8-oxo-GDP) + phosphate. 8-oxo-7,8-dihydroguanosine triphosphate (8-oxo-GTP) is the oxidised form of the free guanine nucleotide and can act as a potent mutagenic substrate for transcription. References: PMID:15878881 Sources: RHEA:60032 Relationships: is a type of nucleoside triphosphate diphosphatase activity [GO:0047429]